{
  "gene": "UniProtKB:Q96S66",
  "gene_symbol": "CLCC1",
  "gene_name": "Chloride channel CLIC-like protein 1",
  "term_id": "GO:0016020",
  "term_label": "membrane"
}